{
  "gene_symbol": "ESRP1",
  "gene_name": "Epithelial splicing regulatory protein 1",
  "term_id": "GO:1990904",
  "term_label": "ribonucleoprotein complex",
  "gene": "UniProtKB:Q6NXG1"
}